dextransucrase activity [GO:0047849] (molecular function) Sources: RHEA:18825 Also known as: CEP, SGE, sucrose 6-glucosyltransferase activity, sucrose-1,6-alpha-glucan glucosyltransferase activity, sucrose:1,6-alpha-D-glucan 6-alpha-D-glucosyltransferase activity Relationships: is a type of GO:0016758 Definition: Catalysis of the reaction: [(1->6)-alpha-D-glucosyl](n) + sucrose = [(1->6)-alpha-D-glucosyl](n+1) + D-fructose.